{
  "gene_name": "Ankyrin repeat domain-containing protein 26",
  "term_id": "UNKNOWN:0003",
  "gene_symbol": "ANKRD26",
  "gene": "UniProtKB:Q9UPS8",
  "term_label": "Unknown cellular component"
}